{
  "gene_symbol": "MAEL",
  "gene_name": "Protein maelstrom homolog",
  "term_label": "male meiotic nuclear division",
  "gene": "UniProtKB:Q96JY0",
  "term_id": "GO:0007140"
}